L-citrulline catabolic process [GO:0019241] (biological process) Relationships: is a type of citrulline metabolic process [GO:0000052]; is a type of GO:0170044; is a type of alpha-amino acid catabolic process [GO:1901606] Definition: The chemical reactions and pathways resulting in the breakdown of L-citrulline, N5-carbamoyl-L-ornithine, an alpha amino acid not found in proteins. Also known as: citrulline breakdown, citrulline catabolism, citrulline degradation Sources: ISBN:0198506732